Atg8 activating enzyme activity [GO:0019779] (molecular function) Also known as: APG7, APG8 activating enzyme activity Sources: GOC:mah Definition: Catalysis of the activation of the small ubiquitin-related modifier APG8, through the formation of an ATP-dependent high-energy thiolester bond. Relationships: is_a ubiquitin-like modifier activating enzyme activity [GO:0008641]